regulation of ERBB signaling pathway [GO:1901184] (BP) Subtypes: regulation of epidermal growth factor receptor signaling pathway [GO:0042058], negative regulation of ERBB signaling pathway [GO:1901185], positive regulation of ERBB signaling pathway [GO:1901186], regulation of ERBB3 signaling pathway [GO:1905578] Definition: Any process that modulates the frequency, rate or extent of ERBB signaling pathway. Relationships: is a type of regulation of signal transduction [GO:0009966]; regulates ERBB signaling pathway [GO:0038127] Sources: GOC:BHF, GOC:TermGenie Also known as: regulation of EGF receptor family signaling pathway, regulation of ERBB signalling pathway, regulation of ErbB signaling, regulation of EGFR family signaling pathway